ventral spinal cord interneuron specification [GO:0021521] (biological process) Relationships: is a type of neuron fate specification [GO:0048665]; is a type of cell fate specification involved in pattern specification [GO:0060573]; is part of ventral spinal cord interneuron fate commitment [GO:0060579] Definition: The process in which a cell becomes capable of differentiating autonomously into a ventral spinal cord interneuron in an environment that is neutral with respect to the developmental pathway. Sources: GOC:cls, GOC:dgh, GOC:dph, GOC:jid, GO_REF:0000021